transposition [GO:0032196] (biological process) Relationships: is a type of cellular process [GO:0009987] Subtypes: DNA transposition [GO:0006313], GO:0032197 References: PMID:14682279, PMID:25893143 Sources: ISBN:1555812090 Definition: Any process involved in mediating the movement of discrete segments of DNA between nonhomologous sites. For elements that are transcribed as the first step of transposition, the process starts with the transcription of the transposable element, its translation and maturation, and ending with integration into DNA. For elements that are cut out, the process starts with the excision of the donor DNA and integrated into another site.